polynucleotide 5'-hydroxyl-kinase activity [GO:0051731] (molecular function) Relationships: is a type of phosphotransferase activity, alcohol group as acceptor [GO:0016773]; is a type of nucleobase-containing compound kinase activity [GO:0019205] Subtypes: ATP-dependent polynucleotide 5'-hydroxyl-kinase activity [GO:0051734], GTP-dependent polynucleotide 5'-hydroxyl-kinase activity [GO:0051735] Also known as: polynucleotide kinase activity, 5'-dephosphopolynucleotide kinase activity, 5'-hydroxyl polynucleotide kinase activity, polynucleotide 5'-hydroxy-kinase activity, polynucleotide 5'-hydroxyl kinase (phosphorylating) activity, PNK Sources: GOC:curators Definition: Catalysis of the reaction: NTP + 5'-dephosphopolynucleotide = NDP + 5'-phosphopolynucleotide. The polynucleotide may be DNA or RNA.